{
  "gene_symbol": "DYNC2I1",
  "gene_name": "Cytoplasmic dynein 2 intermediate chain 1",
  "term_label": "cytoplasmic dynein complex",
  "gene": "UniProtKB:Q8WVS4",
  "term_id": "GO:0005868"
}